{
  "term_id": "GO:0007099",
  "gene_name": "CDK5 regulatory subunit-associated protein 2",
  "term_label": "centriole replication",
  "gene": "UniProtKB:Q96SN8",
  "gene_symbol": "CDK5RAP2"
}